{
  "gene_symbol": "KDM5B",
  "term_label": "histone H3K4me/H3K4me2/H3K4me3 demethylase activity",
  "term_id": "GO:0034647",
  "gene": "UniProtKB:Q9UGL1",
  "gene_name": "Lysine-specific demethylase 5B"
}